{
  "gene_name": "Collagen alpha-1(V) chain",
  "gene": "UniProtKB:P20908",
  "term_label": "skeletal system morphogenesis",
  "gene_symbol": "COL5A1",
  "term_id": "GO:0048705"
}